{
  "term_id": "GO:0000978",
  "gene_symbol": "KLF8",
  "gene": "UniProtKB:O95600",
  "gene_name": "Krueppel-like factor 8",
  "term_label": "RNA polymerase II cis-regulatory region sequence-specific DNA binding"
}